{
  "gene_symbol": "EREG",
  "gene": "UniProtKB:O14944",
  "term_id": "GO:0008284",
  "term_label": "positive regulation of cell population proliferation",
  "gene_name": "Proepiregulin"
}